sympathetic nervous system development [GO:0048485] (biological process) Definition: The process whose specific outcome is the progression of the sympathetic nervous system over time, from its formation to the mature structure. The sympathetic nervous system is one of the two divisions of the vertebrate autonomic nervous system (the other being the parasympathetic nervous system). The sympathetic preganglionic neurons have their cell bodies in the thoracic and lumbar regions of the spinal cord and connect to the paravertebral chain of sympathetic ganglia. Innervate heart and blood vessels, sweat glands, viscera and the adrenal medulla. Most sympathetic neurons, but not all, use noradrenaline as a post-ganglionic neurotransmitter. Sources: FMA:9906, GOC:jid, GOC:sr Relationships: is a type of system development [GO:0048731]; is part of autonomic nervous system development [GO:0048483]